unicellular trichome branch [GO:0090405] (cellular component) Definition: A cell projection part that is a branch of a unicellular trichome. Sources: GOC:tb, PO:0025537 Note: Unicellular trichome (PO:0025537) is a trichome(PO:0000282) that is a single plant cell (PO:0009002). For a cell that forms a branch of a multicellular trichome, see multicellular trichome branch cell (PO:0025163). Relationships: is a type of cellular anatomical structure [GO:0110165]; is part of cell projection [GO:0042995]; has part GO:0090552